thiolester hydrolase activity [GO:0016790] (molecular function) Relationships: is a type of hydrolase activity, acting on ester bonds [GO:0016788] Sources: EC:3.1.2.- Also known as: thiolesterase activity Definition: Catalysis of the reaction: RCO-SR' + H2O = RCOOH + HSR'. This reaction is the hydrolysis of a thiolester bond, an ester formed from a carboxylic acid and a thiol (i.e., RCO-SR'), such as that found in acetyl-coenzyme A. Subtypes: hydroxyacylglutathione hydrolase activity [GO:0004416], palmitoyl-(protein) hydrolase activity [GO:0008474], acyl-CoA hydrolase activity [GO:0016289], fatty acyl-[ACP] hydrolase activity [GO:0016297], S-formylglutathione hydrolase activity [GO:0018738], [citrate-(pro-3S)-lyase] thiolesterase activity [GO:0047778], glutathione thiolesterase activity [GO:0047951], S-succinylglutathione hydrolase activity [GO:0050273]